{
  "gene_name": "Gamma-parvin",
  "term_label": "actin binding",
  "gene_symbol": "PARVG",
  "gene": "UniProtKB:Q9HBI0",
  "term_id": "GO:0003779"
}